{
  "term_id": "GO:0045944",
  "term_label": "positive regulation of transcription by RNA polymerase II",
  "gene_symbol": "SOX18",
  "gene": "UniProtKB:P35713",
  "gene_name": "Transcription factor SOX-18"
}